{
  "term_id": "GO:0098609",
  "gene_symbol": "ITGAV",
  "term_label": "cell-cell adhesion",
  "gene_name": "Integrin alpha-V",
  "gene": "UniProtKB:P06756"
}